{
  "gene": "UniProtKB:Q7Z5L9",
  "gene_symbol": "IRF2BP2",
  "gene_name": "Interferon regulatory factor 2-binding protein 2",
  "term_label": "nucleus",
  "term_id": "GO:0005634"
}